{
  "term_id": "GO:0000774",
  "gene": "UniProtKB:P34932",
  "gene_symbol": "HSPA4",
  "term_label": "adenyl-nucleotide exchange factor activity",
  "gene_name": "Heat shock 70 kDa protein 4"
}